synaptic vesicle maturation [GO:0016188] (biological process) Relationships: is a type of vesicle organization [GO:0016050]; is a type of developmental maturation [GO:0021700] References: PMID:10099709 Sources: GOC:curators Definition: Steps required to form an initiated synaptic vesicle into a fully formed and transmissible synaptic vesicle.